{
  "gene_symbol": "PAPOLG",
  "gene_name": "Poly(A) polymerase gamma",
  "term_label": "nucleus",
  "gene": "UniProtKB:Q9BWT3",
  "term_id": "GO:0005634"
}